{
  "term_id": "GO:0042645",
  "gene_symbol": "POLDIP2",
  "gene_name": "Polymerase delta-interacting protein 2",
  "term_label": "mitochondrial nucleoid",
  "gene": "UniProtKB:Q9Y2S7"
}